{
  "gene_symbol": "GNAI1",
  "gene": "UniProtKB:P63096",
  "term_id": "GO:0031683",
  "gene_name": "Guanine nucleotide-binding protein G(i) subunit alpha-1",
  "term_label": "G-protein beta/gamma-subunit complex binding"
}